{
  "gene": "UniProtKB:Q9GZT8",
  "term_id": "UNKNOWN:0001",
  "gene_name": "NIF3-like protein 1",
  "term_label": "Unknown molecular function",
  "gene_symbol": "NIF3L1"
}